signal transduction [GO:0007165] (biological process) Regulation: regulated by regulation of signal transduction [GO:0009966]; positively regulated by positive regulation of signal transduction [GO:0009967]; negatively regulated by negative regulation of signal transduction [GO:0009968] Sources: GOC:go_curators, GOC:mtg_signaling_feb11 Subtypes: signal transduction involved in filamentous growth [GO:0001402], immune response-regulating signaling pathway [GO:0002764], cell surface receptor signaling pathway [GO:0007166], G protein-coupled receptor signaling pathway [GO:0007186], serotonin receptor signaling pathway [GO:0007210], phototransduction [GO:0007602], hormone-mediated signaling pathway [GO:0009755], carbohydrate mediated signaling [GO:0009756], salicylic acid mediated signaling pathway [GO:0009863], red or far-red light signaling pathway [GO:0010017], regulation of blood pressure by chemoreceptor signaling pathway [GO:0010850], signal transduction involved in regulation of gene expression [GO:0023019], GO:0023041, signal transduction involved in positive regulation of conjugation with cellular fusion [GO:0032005], GO:0035556, signal transduction in absence of ligand [GO:0038034], GO:0038183, lipoprotein particle mediated signaling [GO:0055095], GO:0060863, GO:0071588, sphingolipid mediated signaling pathway [GO:0090520], apoptotic signaling pathway [GO:0097190], necroptotic signaling pathway [GO:0097527], postsynaptic signal transduction [GO:0098926], presynaptic signal transduction [GO:0098928], extracellular ATP signaling [GO:0106167], GO:0140507, opioid growth factor receptor signaling pathway [GO:0140626], signal transduction involved in cellular response to ammonium ion [GO:1903831], ligand-gated ion channel signaling pathway [GO:1990806] Definition: The cellular process in which a signal is conveyed to trigger a change in the activity or state of a cell. Signal transduction begins with reception of a signal (e.g. a ligand binding to a receptor or receptor activation by a stimulus such as light), or for signal transduction in the absence of ligand, signal-withdrawal or the activity of a constitutively active receptor. Signal transduction ends with regulation of a downstream cellular process, e.g. regulation of transcription or regulation of a metabolic process. Signal transduction covers signaling from receptors located on the surface of the cell and signaling via molecules located within the cell. For signaling between cells, signal transduction is restricted to events at and within the receiving cell. Relationships: is_a GO:0009987; is a type of regulation of cellular process [GO:0050794]; is part of cell communication [GO:0007154]; is part of signaling [GO:0023052]; is part of GO:0051716 Note: Note that signal transduction is defined broadly to include a ligand interacting with a receptor, downstream signaling steps and a response being triggered. A change in form of the signal in every step is not necessary. Note that in many cases the end of this process is regulation of the initiation of transcription. Note that specific transcription factors may be annotated to this term, but core/general transcription machinery such as RNA polymerase should not. Also known as: signaling cascade, signalling cascade, signaling pathway, signalling pathway